{
  "term_label": "cytoplasm",
  "gene_symbol": "TRIM5",
  "gene_name": "Tripartite motif-containing protein 5",
  "term_id": "GO:0005737",
  "gene": "UniProtKB:Q9C035"
}